riboflavin catabolic process [GO:0009232] (biological process) References: PMID:10961912 Sources: GOC:jl Also known as: riboflavin breakdown, riboflavin catabolism, riboflavin degradation, vitamin B2 catabolic process, vitamin B2 catabolism, vitamin G catabolic process, vitamin G catabolism Definition: The chemical reactions and pathways resulting in the breakdown of riboflavin (vitamin B2), the precursor for the coenzymes flavin mononucleotide (FMN) and flavin adenine dinucleotide (FAD). Relationships: is a type of GO:0006771; is_a GO:0042365; is a type of flavin-containing compound catabolic process [GO:0042728]